{
  "term_label": "sodium ion transmembrane transport",
  "term_id": "GO:0035725",
  "gene_symbol": "SCN5A",
  "gene": "UniProtKB:Q14524",
  "gene_name": "Sodium channel protein type 5 subunit alpha"
}